{
  "gene": "UniProtKB:P20036",
  "term_id": "GO:0031902",
  "term_label": "late endosome membrane",
  "gene_symbol": "HLA-DPA1",
  "gene_name": "HLA class II histocompatibility antigen, DP alpha 1 chain"
}